amide transport [GO:0042886] (biological process) Subtypes: peptide pheromone export [GO:0000770], allantoate transport [GO:0015719], allantoin transport [GO:0015720], peptide transport [GO:0015833], urea transport [GO:0015840], biotin transport [GO:0015878], coenzyme A transport [GO:0015880], folic acid transport [GO:0015884], pantothenate transmembrane transport [GO:0015887], cycloheximide transport [GO:0015901], fatty-acyl-CoA transport [GO:0015916], GO:0035627, microcin transport [GO:0042884], chloramphenicol transmembrane transport [GO:0042892], GO:0042893, fosmidomycin transport [GO:0042894], ferrichrome import into cell [GO:0042928], achromobactin transport [GO:0042935], bacteriocin transport [GO:0043213], methotrexate transport [GO:0051958], phytochelatin transport [GO:0071993], sulfathiazole transmembrane transport [GO:1902599], 5-amino-1-ribofuranosylimidazole-4-carboxamide transmembrane transport [GO:1903088], asparagine transmembrane transport [GO:1903713], carcinine import across plasma membrane [GO:1905130], GO:1905136, microcystin transport [GO:1905431] Relationships: is a type of nitrogen compound transport [GO:0071705] Definition: The directed movement of an amide, any compound containing one, two, or three acyl groups attached to a nitrogen atom, into, out of or within a cell, or between cells, by means of some agent such as a transporter or pore. Sources: GOC:jl, ISBN:0198506732